{
  "term_id": "GO:0004888",
  "term_label": "transmembrane signaling receptor activity",
  "gene_symbol": "CLEC12A",
  "gene_name": "C-type lectin domain family 12 member A",
  "gene": "UniProtKB:Q5QGZ9"
}